{
  "gene": "UniProtKB:Q01453",
  "gene_name": "Peripheral myelin protein 22",
  "term_id": "GO:0032288",
  "gene_symbol": "PMP22",
  "term_label": "myelin assembly"
}